{
  "term_label": "Ndc80 complex",
  "term_id": "GO:0031262",
  "gene_name": "Kinetochore protein Spc25",
  "gene_symbol": "SPC25",
  "gene": "UniProtKB:Q9HBM1"
}